{
  "term_label": "actin binding",
  "gene": "UniProtKB:Q8IZ21",
  "term_id": "GO:0003779",
  "gene_symbol": "PHACTR4",
  "gene_name": "Phosphatase and actin regulator 4"
}